galectin lattice [GO:0140366] (cellular component) Definition: A non-stoichiometric protein complex formed by several galectins crosslinking glycosylated ligands to form a dynamic lattice. The galectin lattice modulates receptor kinase signaling and the functionality of membrane receptors, by regulating the diffusion, compartmentalization and endocytosis of plasma membrane glycoproteins and glycolipids. References: PMID:19021578, PMID:26092931, PMID:28893908, PMID:30951647 Relationships: is_a GO:0098635